{
  "gene_symbol": "AQP6",
  "term_label": "Unknown cellular component",
  "term_id": "UNKNOWN:0003",
  "gene_name": "Aquaporin-6",
  "gene": "UniProtKB:Q13520"
}